{
  "gene_name": "Laminin subunit beta-1",
  "gene": "UniProtKB:P07942",
  "gene_symbol": "LAMB1",
  "term_id": "GO:0034446",
  "term_label": "substrate adhesion-dependent cell spreading"
}